{
  "gene_symbol": "MAG",
  "gene": "UniProtKB:P20916",
  "term_id": "GO:0005886",
  "term_label": "plasma membrane",
  "gene_name": "Myelin-associated glycoprotein"
}